regulation of cardiac muscle cell membrane potential [GO:0086036] (biological process) Relationships: is a type of regulation of membrane potential [GO:0042391] Sources: GOC:BHF, GOC:mtg_cardiac_conduct_nov11 Definition: Any process that modulates the establishment or extent of a membrane potential in a cardiac muscle cell (a cardiomyocyte). A membrane potential is the electric potential existing across any membrane arising from charges in the membrane itself and from the charges present in the media on either side of the membrane.